{
  "gene_symbol": "ZNF302",
  "gene_name": "Zinc finger protein 302",
  "term_label": "RNA polymerase II cis-regulatory region sequence-specific DNA binding",
  "term_id": "GO:0000978",
  "gene": "UniProtKB:Q9NR11"
}